{
  "gene": "UniProtKB:Q9NY59",
  "term_label": "sphingomyelin metabolic process",
  "gene_name": "Sphingomyelin phosphodiesterase 3",
  "term_id": "GO:0006684",
  "gene_symbol": "SMPD3"
}